{
  "term_label": "axon",
  "term_id": "GO:0030424",
  "gene": "UniProtKB:P07949",
  "gene_name": "Proto-oncogene tyrosine-protein kinase receptor Ret",
  "gene_symbol": "RET"
}